nucleic acid transport [GO:0050657] (biological process) Relationships: is a type of nucleobase-containing compound transport [GO:0015931] Sources: GOC:ai, ISBN:0198506732 Subtypes: RNA transport [GO:0050658], GO:0051027 Definition: The directed movement of nucleic acids, single or double-stranded polynucleotides involved in the storage, transmission and transfer of genetic information, into, out of or within a cell, or between cells, by means of some agent such as a transporter or pore.